{
  "term_label": "protein O-linked glycosylation via N-acetyl-galactosamine",
  "term_id": "GO:0016266",
  "gene_symbol": "POMGNT1",
  "gene_name": "Protein O-linked-mannose beta-1,2-N-acetylglucosaminyltransferase 1",
  "gene": "UniProtKB:Q8WZA1"
}